{
  "gene": "UniProtKB:Q8TCE6",
  "term_id": "GO:0005770",
  "gene_name": "DENN domain-containing protein 10",
  "gene_symbol": "DENND10",
  "term_label": "late endosome"
}